{
  "term_id": "GO:0042277",
  "gene_symbol": "TMEM158",
  "gene_name": "Transmembrane protein 158",
  "term_label": "peptide binding",
  "gene": "UniProtKB:Q8WZ71"
}